{
  "gene": "UniProtKB:P10589",
  "gene_symbol": "NR2F1",
  "term_id": "GO:0000978",
  "gene_name": "COUP transcription factor 1",
  "term_label": "RNA polymerase II cis-regulatory region sequence-specific DNA binding"
}